MHC class II biosynthetic process [GO:0045342] (biological process) Relationships: is a type of macromolecule biosynthetic process [GO:0009059] Regulation: regulated by regulation of MHC class II biosynthetic process [GO:0045346]; negatively regulated by GO:0045347; positively regulated by positive regulation of MHC class II biosynthetic process [GO:0045348] Sources: GOC:go_curators Definition: The chemical reactions and pathways resulting in the formation of major histocompatibility protein class II. Also known as: MHC class II anabolism, MHC class II biosynthesis, MHC class II formation, MHC class II synthesis, major histocompatibility complex class II biosynthesis, major histocompatibility complex class II biosynthetic process